mitochondrial DNA metabolic process [GO:0032042] (biological process) Also known as: mitochondrial DNA metabolism, mtDNA metabolic process, mtDNA metabolism Sources: GOC:mah Relationships: is a type of GO:0006259; occurs in mitochondrion [GO:0005739] Definition: The chemical reactions and pathways involving mitochondrial DNA. Regulation: regulated by regulation of mitochondrial DNA metabolic process [GO:1901858]; negatively regulated by GO:1901859; positively regulated by GO:1901860 Subtypes: mitochondrial DNA replication [GO:0006264], mitochondrial DNA catabolic process [GO:0032043], GO:0043504, DNA synthesis involved in mitochondrial DNA replication [GO:0110166], mitochondrion DNA recombination [GO:1905951]